{
  "term_id": "UNKNOWN:0001",
  "gene_name": "Golgi resident protein GCP60",
  "term_label": "Unknown molecular function",
  "gene": "UniProtKB:Q9H3P7",
  "gene_symbol": "ACBD3"
}